cellular response to vitamin B1 [GO:0071301] (biological process) Sources: GOC:mah Relationships: is a type of response to vitamin B1 [GO:0010266]; is a type of GO:0071295; is a type of GO:0097306; is a type of GO:1901699 Definition: Any process that results in a change in state or activity of a cell (in terms of movement, secretion, enzyme production, gene expression, etc.) as a result of a vitamin B1 stimulus. Also known as: cellular response to thiamin, cellular response to thiamine